innate immunity memory response [GO:0090714] (biological process) Definition: An immune response mediated by the innate immune system and directed against a previously encountered immunologic stimulus, being quicker and quantitatively better compared with the initial response to that stimulus. Relationships: is a type of innate immune response [GO:0045087]; is_a immunological memory process [GO:0090713] References: PMID:26086132 Sources: GOC:add Regulation: regulated by regulation of innate immunity memory response [GO:1905680]; RO_0002212 by negative regulation of innate immunity memory response [GO:1905681]; positively regulated by positive regulation of innate immunity memory response [GO:1905682]